{
  "term_label": "ATP hydrolysis activity",
  "term_id": "GO:0016887",
  "gene_name": "Katanin p60 ATPase-containing subunit A-like 2",
  "gene": "UniProtKB:Q8IYT4",
  "gene_symbol": "KATNAL2"
}